associative learning [GO:0008306] (biological process) Definition: Learning by associating a stimulus (the cause) with a particular outcome (the effect). Relationships: is a type of learning [GO:0007612] Sources: ISBN:0582227089 Also known as: Pavlovian conditioning, classical conditioning, conditional learning, conditional response Subtypes: conditioned taste aversion [GO:0001661], GO:0008355, GO:0008542, conditioned place preference [GO:1990708]